{
  "gene_symbol": "EXOSC8",
  "term_label": "TRAMP-dependent tRNA surveillance pathway",
  "gene_name": "Exosome complex component RRP43",
  "term_id": "GO:0071038",
  "gene": "UniProtKB:Q96B26"
}